{
  "gene": "UniProtKB:Q7Z3E1",
  "term_label": "NAD+-protein mono-ADP-ribosyltransferase activity",
  "term_id": "GO:1990404",
  "gene_symbol": "TIPARP",
  "gene_name": "Protein mono-ADP-ribosyltransferase TIPARP"
}